{
  "gene": "UniProtKB:Q9HBI5",
  "gene_symbol": "CEP15",
  "gene_name": "Centrosomal protein 15 kDa",
  "term_label": "Unknown molecular function",
  "term_id": "UNKNOWN:0001"
}